peptidoglycan binding [GO:0042834] (MF) References: PMID:14698226 Sources: GOC:go_curators Relationships: is a type of GO:0005539 Definition: Interacting selectively and non-covalently, in a non-covalent manner, with peptidoglycan, any of a class of glycoconjugates found in bacterial cell walls.